{
  "term_id": "GO:0001889",
  "gene_name": "UDP-glucuronosyltransferase 1-6",
  "gene_symbol": "UGT1A6",
  "term_label": "liver development",
  "gene": "UniProtKB:P19224"
}